{
  "term_label": "SCF ubiquitin ligase complex",
  "term_id": "GO:0019005",
  "gene": "UniProtKB:Q9UF56",
  "gene_name": "F-box_LRR-repeat protein 17",
  "gene_symbol": "FBXL17"
}